feruloyl esterase activity [GO:0030600] (molecular function) Relationships: is a type of carboxylic ester hydrolase activity [GO:0052689] Sources: EC:3.1.1.73 Definition: Catalysis of the reaction: feruloyl-polysaccharide + H2O = ferulate + polysaccharide. Also known as: cinnamoyl ester hydrolase activity, 4-hydroxy-3-methoxycinnamoyl-sugar hydrolase activity, FAE-I, FAE-II, FAE-III, FAEA, cinnAE, ferulic acid esterase activity, hemicellulase accessory, hydroxycinnamoyl esterase activity